{
  "gene_symbol": "SERPINA13P",
  "term_id": "GO:0005615",
  "gene": "UniProtKB:Q6UXR4",
  "term_label": "extracellular space",
  "gene_name": "Putative serpin A13"
}